{
  "gene_name": "Metallothionein-1M",
  "term_label": "nucleus",
  "term_id": "GO:0005634",
  "gene": "UniProtKB:Q8N339",
  "gene_symbol": "MT1M"
}